retinol dehydratase activity [GO:0017051] (molecular function) Relationships: is a type of hydro-lyase activity [GO:0016836] References: PMID:9857081 Definition: Catalysis of the reaction: 3'-phosphoadenosine 5'-phosphosulfate + retinol = adenosine 3',5'-bisphosphate + anhydroretinol.